histamine-gated chloride channel activity [GO:0019182] (molecular function) Sources: GOC:mtg_transport, ISBN:0815340729 Relationships: is a type of chloride channel activity [GO:0005254] Definition: Enables the energy-independent facilitated diffusion of a chloride ion through a transmembrane channel that opens when bound to histamine.